{
  "term_label": "intracellular phosphate ion homeostasis",
  "term_id": "GO:0030643",
  "gene_symbol": "SLC34A3",
  "gene_name": "Sodium-dependent phosphate transport protein 2C",
  "gene": "UniProtKB:Q8N130"
}